{
  "gene_symbol": "SYT7",
  "gene_name": "Synaptotagmin-7",
  "gene": "UniProtKB:O43581",
  "term_id": "GO:0006906",
  "term_label": "vesicle fusion"
}